{
  "gene": "UniProtKB:Q9H4Q4",
  "gene_name": "PR domain zinc finger protein 12",
  "term_label": "nucleus",
  "term_id": "GO:0005634",
  "gene_symbol": "PRDM12"
}